{
  "gene_symbol": "MUC4",
  "term_id": "UNKNOWN:0001",
  "term_label": "Unknown molecular function",
  "gene_name": "Mucin-4",
  "gene": "UniProtKB:Q99102"
}